{
  "gene_name": "Cytokine receptor common subunit beta",
  "term_id": "GO:0007259",
  "gene": "UniProtKB:P32927",
  "gene_symbol": "CSF2RB",
  "term_label": "cell surface receptor signaling pathway via JAK-STAT"
}